{
  "gene": "UniProtKB:Q14993",
  "term_label": "extracellular matrix",
  "gene_symbol": "COL19A1",
  "term_id": "GO:0031012",
  "gene_name": "Collagen alpha-1(XIX) chain"
}